{
  "term_label": "obsolete mitochondrial respiratory chain complex IV",
  "term_id": "GO:0005751",
  "gene_symbol": "COX6C",
  "gene": "UniProtKB:P09669",
  "gene_name": "Cytochrome c oxidase subunit 6C"
}